{
  "gene_symbol": "SCPEP1",
  "gene_name": "Retinoid-inducible serine carboxypeptidase",
  "gene": "UniProtKB:Q9HB40",
  "term_label": "serine-type carboxypeptidase activity",
  "term_id": "GO:0004185"
}